{
  "gene_symbol": "PCBP3",
  "term_id": "GO:0005737",
  "gene_name": "Poly(rC)-binding protein 3",
  "gene": "UniProtKB:P57721",
  "term_label": "cytoplasm"
}